{
  "gene": "UniProtKB:Q6P4I2",
  "term_label": "cytosol",
  "gene_symbol": "WDR73",
  "gene_name": "WD repeat-containing protein 73",
  "term_id": "GO:0005829"
}